anterior/posterior axis specification, follicular epithelium [GO:0030714] (biological process) Definition: Polarization of the follicle cells of an insect ovary along the anterior/posterior axis. Sources: GOC:bf Relationships: is a type of developmental process involved in reproduction [GO:0003006]; is a type of GO:0009798; is a type of establishment or maintenance of polarity of follicular epithelium [GO:0016334]; is part of follicle cell of egg chamber development [GO:0030707] Also known as: anterior/posterior axis determination, follicular epithelium